{
  "gene": "UniProtKB:Q9P2J8",
  "gene_name": "Zinc finger protein 624",
  "term_label": "regulation of transcription by RNA polymerase II",
  "term_id": "GO:0006357",
  "gene_symbol": "ZNF624"
}